{
  "gene_symbol": "TERB2",
  "gene": "UniProtKB:Q8NHR7",
  "term_id": "GO:0070197",
  "gene_name": "Telomere repeats-binding bouquet formation protein 2",
  "term_label": "meiotic attachment of telomere to nuclear envelope"
}